{
  "gene_name": "Tripartite motif-containing protein 72",
  "term_label": "ubiquitin protein ligase activity",
  "gene": "UniProtKB:Q6ZMU5",
  "gene_symbol": "TRIM72",
  "term_id": "GO:0061630"
}